{
  "gene_symbol": "PLXNB1",
  "term_id": "GO:0050772",
  "term_label": "positive regulation of axonogenesis",
  "gene_name": "Plexin-B1",
  "gene": "UniProtKB:O43157"
}